{
  "gene_symbol": "ITGB3",
  "gene": "UniProtKB:P05106",
  "term_label": "integrin complex",
  "gene_name": "Integrin beta-3",
  "term_id": "GO:0008305"
}